{
  "gene_symbol": "GDF1",
  "term_id": "GO:0005125",
  "gene": "UniProtKB:P27539",
  "term_label": "cytokine activity",
  "gene_name": "Embryonic growth_differentiation factor 1"
}